{
  "term_id": "GO:0030426",
  "gene_symbol": "CDK5R2",
  "term_label": "growth cone",
  "gene_name": "Cyclin-dependent kinase 5 activator 2",
  "gene": "UniProtKB:Q13319"
}